{
  "term_id": "GO:0005874",
  "term_label": "microtubule",
  "gene_name": "Kinesin-1 heavy chain",
  "gene_symbol": "KIF5B",
  "gene": "UniProtKB:P33176"
}